{
  "gene_symbol": "HMOX2",
  "gene_name": "Heme oxygenase 2",
  "gene": "UniProtKB:P30519",
  "term_id": "GO:0004392",
  "term_label": "heme oxygenase (decyclizing) activity"
}